{
  "gene_symbol": "PATE3",
  "term_id": "UNKNOWN:0002",
  "gene_name": "Prostate and testis expressed protein 3",
  "gene": "UniProtKB:B3GLJ2",
  "term_label": "Unknown biological process"
}